U4 snRNA 3'-end processing [GO:0034475] (biological process) Also known as: U4 snRNA 3' end processing Relationships: is a type of snRNA 3'-end processing [GO:0034472] Definition: Any process involved in forming the mature 3' end of a U4 snRNA molecule. Sources: GOC:mah